{
  "gene_symbol": "KRT10",
  "term_id": "GO:0002009",
  "gene": "UniProtKB:P13645",
  "gene_name": "Keratin, type I cytoskeletal 10",
  "term_label": "morphogenesis of an epithelium"
}